{
  "term_label": "calcium-dependent protein kinase inhibitor activity",
  "term_id": "GO:0008427",
  "gene_name": "Calcium_calmodulin-dependent protein kinase II inhibitor 1",
  "gene": "UniProtKB:Q7Z7J9",
  "gene_symbol": "CAMK2N1"
}